{
  "term_id": "GO:0098038",
  "gene": "UniProtKB:Q8N414",
  "gene_symbol": "PGBD5",
  "gene_name": "PiggyBac transposable element-derived protein 5",
  "term_label": "non-replicative DNA transposition"
}